protein-exporting ATPase activity [GO:0008564] (molecular function) Note: Represents ATP- hydrolyzing enzymes of the general secretory pathway (Sec or Type II), of the virulence-related secretory pathway (Type III) and of the conjugal DNA-protein transfer pathway (Type IV). Type II enzymes occur in bacteria, archaea and eukaryotes, whereas type III and type IV enzymes occur in bacteria where they form components of a multi-subunit complex. Also known as: ATPase-coupled protein transporter activity Definition: Enables the transfer of a solute or solutes from one side of a membrane to the other according to the reaction: ATP + H2O + protein+(in) = ADP + phosphate + protein+(out); drives the concomitant secretion of proteins. References: PMID:30346996 Sources: EC:7.4.2.8 Relationships: is a type of protein-transporting ATPase activity [GO:0015450]